{
  "gene_name": "Serine_threonine-protein phosphatase 2A 55 kDa regulatory subunit B gamma isoform",
  "gene": "UniProtKB:Q9Y2T4",
  "gene_symbol": "PPP2R2C",
  "term_id": "GO:0005829",
  "term_label": "cytosol"
}